{
  "gene_symbol": "SLC35B1",
  "term_id": "GO:0005460",
  "term_label": "UDP-glucose transmembrane transporter activity",
  "gene_name": "Solute carrier family 35 member B1",
  "gene": "UniProtKB:P78383"
}